{
  "gene_name": "Importin subunit alpha-1",
  "term_label": "NLS-dependent protein nuclear import complex",
  "term_id": "GO:0042564",
  "gene": "UniProtKB:P52292",
  "gene_symbol": "KPNA2"
}